FAT10 conjugating enzyme activity [GO:0061652] (molecular function) Sources: GOC:dph Relationships: is_a GO:0019775; is a type of ubiquitin-like protein conjugating enzyme activity [GO:0061650] Also known as: E2 Definition: Isoenergetic transfer of FAT10 from one protein to another via the reaction X-FAT10 + Y = Y-FAT10 + X, where both the X-FAT10 and Y-FAT10 linkages are thioester bonds between the C-terminal amino acid of FAT10 and a sulfhydryl side group of a cysteine residue.